{
  "term_label": "neuron projection",
  "gene_symbol": "FAM107A",
  "gene_name": "Actin-associated protein FAM107A",
  "term_id": "GO:0043005",
  "gene": "UniProtKB:O95990"
}